{
  "term_id": "GO:0005615",
  "gene_symbol": "CD1A",
  "term_label": "extracellular space",
  "gene": "UniProtKB:P06126",
  "gene_name": "T-cell surface glycoprotein CD1a"
}